{
  "term_label": "neuron development",
  "gene_symbol": "ESX1",
  "gene_name": "Homeobox protein ESX1",
  "term_id": "GO:0048666",
  "gene": "UniProtKB:Q8N693"
}